{
  "gene_symbol": "MYH14",
  "term_label": "actomyosin structure organization",
  "term_id": "GO:0031032",
  "gene_name": "Myosin-14",
  "gene": "UniProtKB:Q7Z406"
}